{
  "gene_symbol": "UBA52",
  "term_id": "GO:0022626",
  "term_label": "cytosolic ribosome",
  "gene": "UniProtKB:P62987",
  "gene_name": "Ubiquitin-ribosomal protein eL40 fusion protein"
}